negative regulation of platelet aggregation [GO:0090331] (biological process) Also known as: platelet disaggregation Sources: GOC:BHF Definition: Any process that decreases the rate, frequency or extent of platelet aggregation. Platelet aggregation is the adhesion of one platelet to one or more other platelets via adhesion molecules. Relationships: is a type of negative regulation of platelet activation [GO:0010544]; is a type of negative regulation of homotypic cell-cell adhesion [GO:0034111]; is a type of GO:0090330; RO_0002212 platelet aggregation [GO:0070527]